Rohon-Beard neuron differentiation [GO:1905275] (biological process) Definition: The process in which a relatively unspecialized cell acquires the specialized features of a Rohon-Beard neuron. Sources: GOC:TermGenie, GO_REF:0000086, ZFIN:ZDB-PUB-120807-45 Relationships: is a type of GO:0021953